response to L-cysteine [GO:1901367] (biological process) Subtypes: GO:0036346 Definition: Any process that results in a change in state or activity of a cell or an organism (in terms of movement, secretion, enzyme production, gene expression, etc.) as a result of a L-cysteine stimulus. Relationships: is a type of GO:0043200; is a type of GO:1901698; is a type of response to oxygen-containing compound [GO:1901700] Sources: GOC:TermGenie